{
  "gene_symbol": "BPNT1",
  "term_id": "UNKNOWN:0003",
  "gene": "UniProtKB:O95861",
  "term_label": "Unknown cellular component",
  "gene_name": "3'(2'),5'-bisphosphate nucleotidase 1"
}